ATP deaminase activity [GO:0047692] (molecular function) Definition: Catalysis of the reaction: ATP + H2O = ITP + NH3. Sources: EC:3.5.4.18, MetaCyc:ATP-DEAMINASE-RXN Relationships: is a type of GO:0047623 Also known as: ATP aminohydrolase activity, adenosine triphosphate deaminase activity